{
  "term_label": "delta DNA polymerase complex",
  "gene_symbol": "POLD2",
  "term_id": "GO:0043625",
  "gene_name": "DNA polymerase delta subunit 2",
  "gene": "UniProtKB:P49005"
}